{
  "gene_symbol": "GTF2IRD2B",
  "term_label": "nucleus",
  "gene_name": "General transcription factor II-I repeat domain-containing protein 2B",
  "term_id": "GO:0005634",
  "gene": "UniProtKB:Q6EKJ0"
}